{
  "gene": "UniProtKB:Q9Y3B1",
  "term_id": "GO:1990050",
  "gene_symbol": "PRELID3B",
  "term_label": "phosphatidic acid transfer activity",
  "gene_name": "PRELI domain containing protein 3B"
}